ingression involved in gastrulation with mouth forming second [GO:0055111] (biological process) Definition: The migration of individual cells into the embryo involved in deuterostomic gastrulation. Relationships: is_a cell migration involved in gastrulation [GO:0042074]; is part of GO:0001702 Sources: ISBN:0878932437